{
  "term_label": "auditory receptor cell development",
  "term_id": "GO:0060117",
  "gene": "UniProtKB:Q9Y6M7",
  "gene_name": "Sodium bicarbonate cotransporter 3",
  "gene_symbol": "SLC4A7"
}